response to nonane [GO:1902780] (biological process) Definition: Any process that results in a change in state or activity of a cell or an organism (in terms of movement, secretion, enzyme production, gene expression, etc.) as a result of a nonane stimulus. References: PMID:22958739 Sources: GOC:TermGenie, GOC:mengo_curators, GO_REF:0000071 Relationships: is a type of response to alkane [GO:1902778] Subtypes: cellular response to nonane [GO:1902781]